tRNA stabilization [GO:0036416] (biological process) References: PMID:20459084 Sources: GOC:aa, GOC:bf Relationships: is a type of regulation of tRNA stability [GO:0036415]; is a type of RNA stabilization [GO:0043489]; is a type of negative regulation of tRNA catabolic process [GO:1902371] Definition: Prevention of degradation of tRNA molecules.